negative regulation of nuclear migration along microtubule [GO:1902839] (biological process) Definition: Any process that stops, prevents or reduces the frequency, rate or extent of nuclear migration along microtubule. Relationships: is a type of negative regulation of intracellular transport [GO:0032387]; is a type of GO:1902838; negatively regulates nuclear migration along microtubule [GO:0030473] Also known as: down regulation of microtubule cytoskeleton-dependent nuclear positioning, down regulation of microtubule cytoskeleton-dependent nucleus positioning, down regulation of microtubule-dependent nuclear positioning, down regulation of microtubule-dependent nucleus positioning, down regulation of microtubule-mediated nuclear migration, down regulation of nuclear migration along microtubule, down regulation of nuclear migration, microtubule-mediated, down regulation of transport of nucleus by microtubules, down regulation of transport of nucleus, microtubule-mediated, down-regulation of microtubule cytoskeleton-dependent nuclear positioning, down-regulation of microtubule cytoskeleton-dependent nucleus positioning, down-regulation of microtubule-dependent nuclear positioning, down-regulation of microtubule-dependent nucleus positioning, down-regulation of microtubule-mediated nuclear migration, down-regulation of nuclear migration along microtubule, down-regulation of nuclear migration, microtubule-mediated, down-regulation of transport of nucleus by microtubules, down-regulation of transport of nucleus, microtubule-mediated, downregulation of microtubule cytoskeleton-dependent nuclear positioning, downregulation of microtubule cytoskeleton-dependent nucleus positioning, downregulation of microtubule-dependent nuclear positioning, downregulation of microtubule-dependent nucleus positioning, downregulation of microtubule-mediated nuclear migration, downregulation of nuclear migration along microtubule, downregulation of nuclear migration, microtubule-mediated, downregulation of transport of nucleus by microtubules, downregulation of transport of nucleus, microtubule-mediated, negative regulation of microtubule cytoskeleton-dependent nuclear positioning, negative regulation of microtubule cytoskeleton-dependent nucleus positioning, negative regulation of microtubule-dependent nuclear positioning, negative regulation of microtubule-dependent nucleus positioning, negative regulation of microtubule-mediated nuclear migration, negative regulation of nuclear migration, microtubule-mediated, negative regulation of transport of nucleus by microtubules, negative regulation of transport of nucleus, microtubule-mediated, inhibition of microtubule cytoskeleton-dependent nuclear positioning, inhibition of microtubule cytoskeleton-dependent nucleus positioning, inhibition of microtubule-dependent nuclear positioning, inhibition of microtubule-dependent nucleus positioning, inhibition of microtubule-mediated nuclear migration, inhibition of nuclear migration along microtubule, inhibition of nuclear migration, microtubule-mediated, inhibition of transport of nucleus by microtubules, inhibition of transport of nucleus, microtubule-mediated Subtypes: negative regulation of nuclear migration during mitotic telophase [GO:1902853] References: PMID:23087209 Sources: GOC:TermGenie, GO_REF:0000058